{
  "gene": "UniProtKB:P29401",
  "gene_name": "Transketolase",
  "term_label": "pentose-phosphate shunt, non-oxidative branch",
  "gene_symbol": "TKT",
  "term_id": "GO:0009052"
}